{
  "gene_symbol": "SNRPD3",
  "gene": "UniProtKB:P62318",
  "gene_name": "Small nuclear ribonucleoprotein Sm D3",
  "term_label": "SMN-Sm protein complex",
  "term_id": "GO:0034719"
}